{
  "term_label": "vesicle docking involved in exocytosis",
  "gene_name": "Vacuolar protein sorting-associated protein 11 homolog",
  "gene_symbol": "VPS11",
  "term_id": "GO:0006904",
  "gene": "UniProtKB:Q9H270"
}